determination of muscle attachment site [GO:0016204] (biological process) Definition: The process that mediates the transfer of information from the cells of a muscle to those of its intended target, thereby identifying the target site. Sources: GOC:isa_complete Relationships: is a type of cell-cell signaling [GO:0007267]; is part of GO:0016203